{
  "term_label": "actin cytoskeleton",
  "term_id": "GO:0015629",
  "gene": "UniProtKB:Q96H55",
  "gene_name": "Unconventional myosin-XIX",
  "gene_symbol": "MYO19"
}